response to toluene [GO:1901424] (biological process) Regulation: regulated by regulation of response to toluene [GO:1901454]; negatively regulated by negative regulation of response to toluene [GO:1901455]; positively regulated by positive regulation of response to toluene [GO:1901456] Sources: GOC:TermGenie, GOC:mengo_curators Relationships: is a type of GO:0042221 Definition: Any process that results in a change in state or activity of a cell or an organism (in terms of movement, secretion, enzyme production, gene expression, etc.) as a result of a toluene stimulus.